{
  "term_id": "GO:0005178",
  "term_label": "integrin binding",
  "gene": "UniProtKB:O95388",
  "gene_symbol": "CCN4",
  "gene_name": "CCN family member 4"
}